{
  "term_label": "Unknown cellular component",
  "term_id": "UNKNOWN:0003",
  "gene_symbol": "BEAN1",
  "gene": "UniProtKB:Q3B7T3",
  "gene_name": "Protein BEAN1"
}